{
  "gene_name": "Malignant fibrous histiocytoma-amplified sequence 1",
  "gene_symbol": "MFHAS1",
  "gene": "UniProtKB:Q9Y4C4",
  "term_label": "Unknown molecular function",
  "term_id": "UNKNOWN:0001"
}